sensory epithelium regeneration [GO:0070654] (biological process) References: PMID:19381250 Sources: GOC:dsf Subtypes: mechanosensory epithelium regeneration [GO:0070655] Relationships: is a type of epithelium regeneration [GO:1990399] Definition: The regrowth of a sensory epithelium following its loss or destruction.